{
  "term_id": "UNKNOWN:0003",
  "gene": "UniProtKB:Q8IZ73",
  "term_label": "Unknown cellular component",
  "gene_name": "Pseudouridylate synthase RPUSD2",
  "gene_symbol": "RPUSD2"
}